{
  "term_id": "GO:0051301",
  "term_label": "cell division",
  "gene_symbol": "SPART",
  "gene_name": "Spartin",
  "gene": "UniProtKB:Q8N0X7"
}